{
  "gene_symbol": "TRBV5-8",
  "term_label": "plasma membrane",
  "gene_name": "T cell receptor beta variable 5-8",
  "gene": "UniProtKB:A0A5A2",
  "term_id": "GO:0005886"
}